prolactin receptor binding [GO:0005148] (molecular function) Also known as: prolactin, prolactin receptor ligand Definition: Binding to a prolactin receptor. Relationships: is a type of cytokine receptor binding [GO:0005126] Sources: GOC:ai